{
  "gene_name": "Semaphorin-6C",
  "term_id": "GO:0071526",
  "gene": "UniProtKB:Q9H3T2",
  "gene_symbol": "SEMA6C",
  "term_label": "semaphorin-plexin signaling pathway"
}